choriogonadotropin hormone binding [GO:0038106] (molecular function) Also known as: chorionic gonadotrophin binding, chorionic gonadotropin binding Definition: Binding to choriogonadotropin hormone, a heterodimer, with an alpha subunit identical to that of luteinizing hormone (LH), follicle-stimulating hormone (FSH) and thyroid-stimulating hormone (TSH), and a unique beta subunit. Sources: GOC:BHF, GOC:rl, Wikipedia:Human_chorionic_gonadotropin Relationships: is a type of GO:0042562